negative regulation of gliogenesis [GO:0014014] (biological process) Definition: Any process that stops, prevents, or reduces the frequency, rate or extent of gliogenesis, the formation of mature glia. Sources: GOC:ef Relationships: is a type of GO:0014013; is a type of GO:0050768; negatively regulates GO:0042063 Also known as: down regulation of gliogenesis, down-regulation of gliogenesis, downregulation of gliogenesis, inhibition of gliogenesis Subtypes: GO:0045686, negative regulation of glial cell proliferation [GO:0060253], GO:0070446